acrosomal vesicle exocytosis [GO:0060478] (biological process) Relationships: is a type of calcium-ion regulated exocytosis [GO:0017156]; is part of acrosome reaction [GO:0007340] Regulation: regulated by GO:2000367; positively regulated by positive regulation of acrosomal vesicle exocytosis [GO:2000368] Sources: GOC:dph Also known as: acrosome exocytosis, acrosomal granule exocytosis Definition: The calcium ion regulated exocytosis which results in fusion of the acrosomal vesicle with the plasma membrane of the sperm as part of the acrosome reaction.